{
  "term_label": "Unknown molecular function",
  "gene_symbol": "UBXN6",
  "gene": "UniProtKB:Q9BZV1",
  "term_id": "UNKNOWN:0001",
  "gene_name": "UBX domain-containing protein 6"
}